{
  "gene": "UniProtKB:O60684",
  "term_id": "GO:0042564",
  "gene_name": "Importin subunit alpha-7",
  "gene_symbol": "KPNA6",
  "term_label": "NLS-dependent protein nuclear import complex"
}